{
  "term_label": "peroxisomal membrane",
  "term_id": "GO:0005778",
  "gene_symbol": "PEX12",
  "gene_name": "Peroxisome assembly protein 12",
  "gene": "UniProtKB:O00623"
}